{
  "term_id": "GO:0015140",
  "term_label": "malate transmembrane transporter activity",
  "gene": "UniProtKB:Q9UBX3",
  "gene_symbol": "SLC25A10",
  "gene_name": "Mitochondrial dicarboxylate carrier"
}